{
  "gene_name": "Secretoglobin family 1C member 2",
  "term_id": "UNKNOWN:0001",
  "term_label": "Unknown molecular function",
  "gene_symbol": "SCGB1C2",
  "gene": "UniProtKB:P0DMR2"
}